cellular anatomical structure [GO:0110165] (cellular component) Definition: A part of a cellular organism consisting of a material entity with granularity above the level of a protein complex but below that of an anatomical system. Note that cellular organisms exclude viruses. Subtypes: GO:0000242, cellular bud neck septin structure [GO:0000399], phagophore assembly site [GO:0000407], GO:0000785, GO:0000800, GO:0000801, transverse filament [GO:0000802], spindle pole [GO:0000922], retrotransposon nucleocapsid [GO:0000943], mating projection base [GO:0001400], fibrillar center [GO:0001650], dense fibrillar component [GO:0001651], granular component [GO:0001652], photoreceptor outer segment [GO:0001750], immunological synapse [GO:0001772], GO:0001891, photoreceptor inner segment [GO:0001917], stereocilia coupling link [GO:0002139], GO:0002177, extracellular region [GO:0005576], extracellular space [GO:0005615], cellular bud scar [GO:0005621], GO:0005622, GO:0005630, chitosan layer of spore wall [GO:0005631], inner layer of spore wall [GO:0005632], nuclear lamina [GO:0005652], nucleoplasm [GO:0005654], replication fork [GO:0005657], polytene chromosome weak point [GO:0005702], polytene chromosome ectopic fiber [GO:0005706], chiasma [GO:0005712], recombination nodule [GO:0005713], perichromatin fibrils [GO:0005726], GO:0005737, microtubule organizing center [GO:0005815], intermediate layer of spindle pole body [GO:0005821], inner plaque of spindle pole body [GO:0005822], central plaque of spindle pole body [GO:0005823], GO:0005824, half bridge of spindle pole body [GO:0005825], cytosol [GO:0005829], axoneme [GO:0005930], GO:0005933, nucleoid [GO:0009295], pilus shaft [GO:0009418], GO:0009419, bacterial-type flagellum filament [GO:0009420], GO:0009421, bacterial-type flagellum hook-filament junction [GO:0009422], bacterial-type flagellum hook [GO:0009424], bacterial-type flagellum basal body [GO:0009425], bacterial-type flagellum basal body, distal rod [GO:0009426], bacterial-type flagellum basal body, distal rod, L ring [GO:0009427], bacterial-type flagellum basal body, distal rod, P ring [GO:0009428], GO:0009429, GO:0009431, bacterial-type flagellum basal body, C ring [GO:0009433], GO:0009504, plasmodesmatal desmotubule [GO:0009510], phragmoplast [GO:0009524], phragmosome [GO:0009525], plastid stroma [GO:0009532], etioplast prolamellar body [GO:0009541], granum [GO:0009542], plasmodesmatal cytoplasmic sleeve [GO:0009546], GO:0009548, cellulose microfibril [GO:0009549], preprophase band [GO:0009574], longitudinal side of cell surface [GO:0009930], cell surface [GO:0009986], plastoglobule [GO:0010287], stromule [GO:0010319], external side of cell wall [GO:0010339], GO:0012505, C zone [GO:0014705], longitudinal sarcoplasmic reticulum [GO:0014801], membrane [GO:0016020], lateral plasma membrane [GO:0016328], nuclear matrix [GO:0016363], GO:0019898, GO:0020003, symbiont-containing vacuolar membrane network [GO:0020006], apical complex [GO:0020007], rhoptry [GO:0020008], GO:0020010, ciliary pocket [GO:0020016], kinetoplast [GO:0020023], polar ring of apical complex [GO:0020031], GO:0020032, subpellicular network [GO:0020038], pellicle [GO:0020039], sarcomere [GO:0030017], GO:0030018, GO:0030054, GO:0030061, external encapsulating structure [GO:0030312], GO:0030313, T-tubule [GO:0030315], site of polarized growth [GO:0030427], cell septum [GO:0030428], actin cap [GO:0030478], smooth muscle dense body [GO:0030486], GO:0030496, GO:0030694, rDNA protrusion [GO:0030875], cell leading edge [GO:0031252], cell trailing edge [GO:0031254], GO:0031256, GO:0031257, M band [GO:0031430], GO:0031592, A band [GO:0031672], H zone [GO:0031673], I band [GO:0031674], cytostome [GO:0031910], cytoproct [GO:0031911], oral apparatus [GO:0031912], organelle envelope [GO:0031967], GO:0031974, thylakoid lumen [GO:0031977], organelle subcompartment [GO:0031984], deep fiber [GO:0032123], eisosome [GO:0032126], GO:0032153, septin band [GO:0032158], GO:0032161, medial membrane band [GO:0032178], germ tube [GO:0032179], stereocilium tip [GO:0032426], actin filament bundle [GO:0032432], GO:0032433, cuticular plate [GO:0032437], apical lamina of hyaline layer [GO:0032579], growth cone membrane [GO:0032584], GO:0033012, cellular bud membrane [GO:0033101], cytoskeletal calyx [GO:0033150], gas vesicle shell [GO:0033172], node of Ranvier [GO:0033268], internode region of axon [GO:0033269], paranode region of axon [GO:0033270], basal labyrinth [GO:0033774], nuclear periphery [GO:0034399], centriolar satellite [GO:0034451], organelle-enclosing lipid monolayer [GO:0034646], microtubule organizing center attachment site [GO:0034992], GO:0035182, female germline ring canal inner rim [GO:0035183], ciliary rootlet [GO:0035253], sperm fibrous sheath [GO:0035686], myelin sheath abaxonal region [GO:0035748], myelin sheath adaxonal region [GO:0035749], endonuclear canal [GO:0035843], GO:0035869, scintillon [GO:0036007], acroblast [GO:0036063], hyaluranon cable [GO:0036117], pairing center [GO:0036224], myofilament [GO:0036379], keratohyalin granule [GO:0036457], somatodendritic compartment [GO:0036477], glycogen granule [GO:0042587], GO:0042597, actomyosin [GO:0042641], plasma membrane-derived chromatophore [GO:0042716], yolk granule [GO:0042718], GO:0042763, cell projection [GO:0042995], GO:0043034, GO:0043036, acrosomal matrix [GO:0043159], GO:0043188, GO:0043194, varicosity [GO:0043196], dendritic shaft [GO:0043198], axon hillock [GO:0043203], GO:0043204, myelin sheath [GO:0043209], compact myelin [GO:0043218], lateral loop [GO:0043219], Schmidt-Lanterman incisure [GO:0043220], organelle [GO:0043226], GO:0043245, exosporium [GO:0043592], endospore coat [GO:0043593], endospore cortex [GO:0043595], peribacteroid fluid [GO:0043662], exine [GO:0043668], ectexine [GO:0043669], foot layer [GO:0043670], endexine [GO:0043671], GO:0043672, sexine [GO:0043673], columella [GO:0043674], GO:0043675, tectum [GO:0043676], intine [GO:0043678], filiform apparatus [GO:0043680], polar tube [GO:0044099], nucleoplasmic reticulum [GO:0044195], other organism part [GO:0044217], juxtaparanode region of axon [GO:0044224], GO:0044232, GO:0044280, mitochondrial intracristal space [GO:0044290], dendrite terminus [GO:0044292], GO:0044297, GO:0044298, GO:0044303, main axon [GO:0044304], neuron projection terminus [GO:0044306], endoplasmic reticulum quality control compartment [GO:0044322], dendritic spine neck [GO:0044326], dendritic spine head [GO:0044327], fusome [GO:0045169], intercellular bridge [GO:0045171], apical part of cell [GO:0045177], basal part of cell [GO:0045178], intracellular canaliculus [GO:0046691], dense nuclear body [GO:0046818], GO:0046868, pectic matrix [GO:0048217], GO:0048222, hemicellulose network [GO:0048223], GO:0048224, suberin network [GO:0048225], GO:0048226, perinuclear region of cytoplasm [GO:0048471], presynaptic active zone [GO:0048786], GO:0051233, symplast [GO:0055044], striated muscle dense body [GO:0055120], surface coat of collagen and cuticulin-based cuticle extracellular matrix [GO:0060104], epicuticle of collagen and cuticulin-based cuticle extracellular matrix [GO:0060105], cortical layer of collagen and cuticulin-based cuticle extracellular matrix [GO:0060106], annuli extracellular matrix [GO:0060107], annular furrow extracellular matrix [GO:0060108], medial layer of collagen and cuticulin-based cuticle extracellular matrix [GO:0060109], basal layer of collagen and cuticulin-based cuticle extracellular matrix [GO:0060110], GO:0060111, cell pole [GO:0060187], GO:0060417, yolk plasma [GO:0060418], endocytic patch [GO:0061645], ciliary cap [GO:0061822], GO:0061823, podosome core [GO:0061825], podosome ring [GO:0061826], sperm head [GO:0061827], GO:0061830, actin filament branch point [GO:0061834], ventral surface of cell [GO:0061835], neuron projection branch point [GO:0061845], phagophore [GO:0061908], pollen aperture [GO:0062074], GO:0062160, actin wave [GO:0062201], prospore membrane spindle pole body attachment site [GO:0070057], organellar chromatophore intermembrane space [GO:0070115], inner membrane pellicle complex [GO:0070258], Ubisch body [GO:0070645], GO:0070687, mucus layer [GO:0070701], chrorion micropyle [GO:0070825], sperm individualization complex [GO:0070864], GO:0070865, GO:0070938, GO:0070971, medial cortical node [GO:0071341], cellular birth scar [GO:0071597], satellite fibril [GO:0071808], cell periphery [GO:0071944], ascus epiplasm [GO:0072324], GO:0072562, extrahaustorial matrix [GO:0085036], unicellular trichome branch [GO:0090405], Flemming body [GO:0090543], unicellular trichome apex [GO:0090552], unicellular trichome tip [GO:0090553], extracellular core region of desmosome [GO:0090635], outer dense plaque of desmosome [GO:0090636], inner dense plaque of desmosome [GO:0090637], microsporidian-type endospore [GO:0090641], microsporidian-type exospore [GO:0090642], apical cytoplasm [GO:0090651], basolateral cytoplasm [GO:0090652], cone matrix sheath [GO:0090658], GO:0090688, cleavage furrow leading edge [GO:0090689], mitochondrial membrane scission site [GO:0090692], central region of growth cone [GO:0090724], peripheral region of growth cone [GO:0090725], cortical dynamic polarity patch [GO:0090726], GO:0090734, mitochondrial inner boundary membrane [GO:0097002], perinuclear endoplasmic reticulum [GO:0097038], GO:0097047, GO:0097197, phagocytic cup lip [GO:0097203], GO:0097204, GO:0097217, GO:0097218, sperm midpiece [GO:0097225], sperm mitochondrial sheath [GO:0097226], sperm annulus [GO:0097227], GO:0097228, sperm end piece [GO:0097229], bacterial biofilm matrix surface [GO:0097313], perinucleolar compartment [GO:0097356], tubular endosome [GO:0097422], mitochondrion-associated adherens complex [GO:0097423], GO:0097427, GO:0097433, presynaptic active zone dense projection [GO:0097445], spine mat [GO:0097448], GO:0097478, axonemal central pair [GO:0097540], GO:0097541, GO:0097542, ciliary inversin compartment [GO:0097543], ciliary shaft [GO:0097544], GO:0097545, ciliary base [GO:0097546], left lateral basal body pair [GO:0097562], left middle basal body pair [GO:0097563], right lateral basal body pair [GO:0097564], GO:0097565, left tetrad [GO:0097566], right tetrad [GO:0097567], median body [GO:0097568], lateral shield [GO:0097569], lateral part of cell [GO:0097574], ventral disc lateral crest [GO:0097591], ventral disc overlap zone [GO:0097592], GO:0097593, ventral disc dorsal microribbon [GO:0097594], ventral disc crossbridge [GO:0097595], ventral disc supernumerary microtubule array [GO:0097596], cell surface furrow [GO:0097610], dinoflagellate epicone [GO:0097613], dinoflagellate hypocone [GO:0097614], GO:0097653, dinoflagellate apex [GO:0097683], dinoflagellate antapex [GO:0097684], DIM/DIP cell wall layer [GO:0097735], GO:0098552, chromosomal region [GO:0098687], presynapse [GO:0098793], GO:0098794, presynaptic endocytic zone [GO:0098833], postsynaptic endocytic zone [GO:0098843], GO:0098862, actin body [GO:0099079], supramolecular complex [GO:0099080], GO:0099086, reservosome lumen [GO:0106124], reservosome matrix [GO:0106125], GO:0106126, cellularization cleavage furrow invagination front [GO:0110071], nucleus leading edge [GO:0110092], nucleus lagging edge [GO:0110093], stereocilium shaft [GO:0120043], GO:0120044, smooth endoplasmic reticulum cisterna [GO:0120082], rough endoplasmic reticulum cisterna [GO:0120083], procentriole [GO:0120098], GO:0120100, bacterial-type flagellum secretion apparatus [GO:0120102], GO:0120104, mitotic actomyosin contractile ring, intermediate layer [GO:0120105], mitotic actomyosin contractile ring, distal actin filament layer [GO:0120106], bacterial-type flagellum rotor complex [GO:0120107], bilobe structure [GO:0120120], tripartite attachment complex [GO:0120121], proximal portion of axoneme [GO:0120134], distal portion of axoneme [GO:0120135], photoreceptor proximal connecting cilium [GO:0120205], GO:0120206, sperm head-tail coupling apparatus [GO:0120212], subapical part of cell [GO:0120219], basal body patch [GO:0120220], ciliary microtubule quartet [GO:0120260], GO:0120280, Hechtian strand [GO:0120307], nuclear envelope adjacent to nuclear pore complex [GO:0120321], cnida [GO:0140022], mitotic nuclear bridge [GO:0140510], mitotic nuclear bridge stalk [GO:0140511], mitotic nuclear bridge midzone [GO:0140512], GO:0140599, GO:0140918, GO:0150004, distal axon [GO:0150034], axonemal microtubule doublet inner sheath [GO:0160110], axonemal A tubule inner sheath [GO:0160111], axonemal B tubule inner sheath [GO:0160112], axonemal microtubule doublet inner junction [GO:0160113], axonemal microtubule doublet outer junction [GO:0160114], axonemal microtubule doublet ribbon [GO:0160115], meisosome [GO:0160132], polar tube anchoring disc [GO:0160202], pyrenoid tubule [GO:0160223], endoplasmic reticulum membrane-lipid droplet contact site [GO:0160259], GO:0170047, presynaptic grid [GO:1990013], orthogonal array [GO:1990014], GO:1990015, neck portion of tanycyte [GO:1990016], tail portion of tanycyte [GO:1990018], pericellular basket [GO:1990030], pinceau fiber [GO:1990031], GO:1990037, Lewy body corona [GO:1990038], GO:1990047, perforation plate [GO:1990073], rhoptry neck [GO:1990225], GO:1990295, stereocilia tip-link density [GO:1990427], axonemal central apparatus [GO:1990716], axonemal central bridge [GO:1990717], axonemal central pair projection [GO:1990718], microtubule end [GO:1990752], GO:1990783, basolateral part of cell [GO:1990794], GO:1990805, mating projection actin fusion focus [GO:1990819], nucleoplasmic periphery of the nuclear pore complex [GO:1990826], lysosomal matrix [GO:1990836], nucleoplasmic side of nuclear pore [GO:1990875], GO:1990876, ciliary pocket collar [GO:1990900], Isp3 layer of spore wall [GO:1990916] Sources: GOC:kmv Relationships: is a type of cellular_component [GO:0005575] Also known as: cellular anatomical entity